eoxin C4 synthase activity [GO:0097261] (molecular function) References: PMID:18184802, PMID:18647347 Sources: GOC:mw Definition: Catalysis of the reaction: eoxin A4 + glutathione = eoxin C4. Relationships: is a type of GO:0016846